{
  "gene": "UniProtKB:Q9Y678",
  "term_label": "intra-Golgi vesicle-mediated transport",
  "gene_name": "Coatomer subunit gamma-1",
  "term_id": "GO:0006891",
  "gene_symbol": "COPG1"
}